positive regulation of cell wall organization or biogenesis [GO:1903340] (biological process) Subtypes: positive regulation of secondary cell wall biogenesis [GO:1901348] Definition: Any process that activates or increases the frequency, rate or extent of cell wall organization or biogenesis. Relationships: is a type of GO:0048522; is a type of GO:1903338; positively regulates cell wall organization or biogenesis [GO:0071554] Sources: GOC:TermGenie, GOC:vw, GO_REF:0000058 Also known as: positive regulation of cell wall organisation or biogenesis, positive regulation of cell wall organization or biogenesis at cellular level, positive regulation of cellular cell wall organisation or biogenesis, positive regulation of cellular cell wall organization or biogenesis, up regulation of cell wall organisation or biogenesis, up regulation of cell wall organization or biogenesis, up regulation of cell wall organization or biogenesis at cellular level, up regulation of cellular cell wall organisation or biogenesis, up regulation of cellular cell wall organization or biogenesis, up-regulation of cell wall organisation or biogenesis, up-regulation of cell wall organization or biogenesis, up-regulation of cell wall organization or biogenesis at cellular level, up-regulation of cellular cell wall organisation or biogenesis, up-regulation of cellular cell wall organization or biogenesis, upregulation of cell wall organisation or biogenesis, upregulation of cell wall organization or biogenesis, upregulation of cell wall organization or biogenesis at cellular level, upregulation of cellular cell wall organisation or biogenesis, upregulation of cellular cell wall organization or biogenesis, activation of cell wall organisation or biogenesis, activation of cell wall organization or biogenesis, activation of cell wall organization or biogenesis at cellular level, activation of cellular cell wall organisation or biogenesis, activation of cellular cell wall organization or biogenesis